axonemal central apparatus assembly [GO:1904158] (biological process) Definition: The aggregation, arrangement and bonding together of a set of components to form an axonemal central apparatus. References: PMID:9295136 Sources: GOC:TermGenie, GOC:cilia, GOC:krc, GO_REF:0000079 Also known as: axonemal central apparatus formation Relationships: is a type of cellular component assembly [GO:0022607]; is part of axoneme assembly [GO:0035082]